{
  "term_id": "GO:0007166",
  "gene_symbol": "MS4A10",
  "gene": "UniProtKB:Q96PG2",
  "term_label": "cell surface receptor signaling pathway",
  "gene_name": "Membrane-spanning 4-domains subfamily A member 10"
}